{
  "gene": "UniProtKB:P08123",
  "gene_name": "Collagen alpha-2(I) chain",
  "gene_symbol": "COL1A2",
  "term_label": "skeletal system development",
  "term_id": "GO:0001501"
}